symbiont-mediated cell-to-cell migration in host [GO:0106259] (biological process) Definition: The directional movement of a symbiont from one host cell to another. References: PMID:18456802, PMID:19262673, PMID:19816653, PMID:29567712 Sources: GOC:vw Relationships: is_a migration in host [GO:0044001] Subtypes: symbiont-mediated actin polymerization-dependent cell-to-cell migration in host [GO:0070360], symbiont-mediated cell-to-cell migration by invasive hypha [GO:0140649] Also known as: cell-to-cell migration in host, symbiont-mediated dissemination across host cells